{
  "gene_symbol": "BHLHE23",
  "gene": "UniProtKB:Q8NDY6",
  "gene_name": "Class E basic helix-loop-helix protein 23",
  "term_label": "sensory organ development",
  "term_id": "GO:0007423"
}